{
  "gene_symbol": "OTULINL",
  "term_label": "Unknown biological process",
  "gene_name": "Inactive ubiquitin thioesterase OTULINL",
  "term_id": "UNKNOWN:0002",
  "gene": "UniProtKB:Q9NUU6"
}